{
  "gene_name": "Sorting nexin-18",
  "term_label": "cytoplasmic vesicle",
  "gene_symbol": "SNX18",
  "term_id": "GO:0031410",
  "gene": "UniProtKB:Q96RF0"
}